lysine biosynthetic process via diaminopimelate [GO:0009089] (biological process) Definition: The chemical reactions and pathways resulting in the formation of lysine, via the intermediate diaminopimelate. Also known as: diaminopimelate pathway, diaminopimelic acid pathway, lysine anabolism via diaminopimelate, lysine biosynthesis via diaminopimelic acid, lysine biosynthetic process via diaminopimelic acid, lysine formation via diaminopimelate, lysine synthesis via diaminopimelate Sources: GOC:go_curators Subtypes: lysine biosynthetic process via diaminopimelate and N-succinyl-2-amino-6-ketopimelate [GO:0033359], GO:0033360, lysine biosynthetic process via diaminopimelate, dehydrogenase pathway [GO:0033361], lysine biosynthetic process via diaminopimelate, diaminopimelate-aminotransferase pathway [GO:0033362] Relationships: is a type of lysine biosynthetic process [GO:0009085]